{
  "gene": "UniProtKB:A6NK02",
  "gene_name": "Tripartite motif-containing protein 75",
  "term_label": "ubiquitin protein ligase activity",
  "term_id": "GO:0061630",
  "gene_symbol": "TRIM75"
}